{
  "term_id": "UNKNOWN:0003",
  "term_label": "Unknown cellular component",
  "gene_symbol": "NXPE3",
  "gene": "UniProtKB:Q969Y0",
  "gene_name": "NXPE family member 3"
}